{
  "gene": "UniProtKB:Q2NL82",
  "term_label": "nucleolus",
  "term_id": "GO:0005730",
  "gene_name": "Pre-rRNA-processing protein TSR1 homolog",
  "gene_symbol": "TSR1"
}